{
  "gene": "UniProtKB:P46663",
  "term_label": "plasma membrane",
  "gene_symbol": "BDKRB1",
  "term_id": "GO:0005886",
  "gene_name": "B1 bradykinin receptor"
}